dopamine catabolic process [GO:0042420] (BP) Definition: The chemical reactions and pathways resulting in the breakdown of dopamine, a catecholamine neurotransmitter and a metabolic precursor of noradrenaline and adrenaline. Sources: GOC:jl, ISBN:0198506732 Relationships: is a type of dopamine metabolic process [GO:0042417]; is a type of GO:0042424 Also known as: dopamine breakdown, dopamine catabolism, dopamine degradation